{
  "gene_name": "V(D)J recombination-activating protein 1",
  "term_label": "V(D)J recombination",
  "gene_symbol": "RAG1",
  "gene": "UniProtKB:P15918",
  "term_id": "GO:0033151"
}